{
  "gene": "UniProtKB:P58005",
  "term_id": "GO:0016684",
  "term_label": "oxidoreductase activity, acting on peroxide as acceptor",
  "gene_name": "Sestrin-3",
  "gene_symbol": "SESN3"
}